auditory receptor cell fate specification [GO:0042667] (biological process) Also known as: auditory hair cell fate specification Definition: The process in which a cell becomes capable of differentiating autonomously into an auditory hair cell in an environment that is neutral with respect to the developmental pathway; upon specification, the cell fate can be reversed. Relationships: is a type of GO:0048665; is part of auditory receptor cell fate commitment [GO:0009912] Regulation: RO_0002212 by negative regulation of auditory receptor cell fate specification [GO:0009999]; regulated by regulation of inner ear auditory receptor cell fate specification [GO:0042669] Sources: GOC:go_curators